{
  "term_label": "Unknown cellular component",
  "gene_name": "Myotubularin-related protein 14",
  "term_id": "UNKNOWN:0003",
  "gene_symbol": "MTMR14",
  "gene": "UniProtKB:Q8NCE2"
}